{
  "gene": "UniProtKB:P82970",
  "term_label": "Unknown biological process",
  "gene_name": "High mobility group nucleosome-binding domain-containing protein 5",
  "term_id": "UNKNOWN:0002",
  "gene_symbol": "HMGN5"
}